{
  "gene_name": "Olfactory receptor 4K14",
  "gene_symbol": "OR4K14",
  "gene": "UniProtKB:Q8NGD5",
  "term_label": "Unknown cellular component",
  "term_id": "UNKNOWN:0003"
}